{
  "gene": "UniProtKB:Q99504",
  "gene_symbol": "EYA3",
  "gene_name": "Eyes absent homolog 3",
  "term_label": "negative regulation of extrinsic apoptotic signaling pathway in absence of ligand",
  "term_id": "GO:2001240"
}